response to prolactin [GO:1990637] (biological process) References: PMID:7760850 Definition: Any process that results in a change in state or activity of a cell or an organism (in terms of movement, secretion, enzyme production, gene expression, etc.) as a result of a prolactin stimulus. The anterior pituitary hormone prolactin has a number of roles including being essential for lactation. Subtypes: GO:1990646 Relationships: is a type of response to peptide hormone [GO:0043434]